{
  "term_label": "neuron projection",
  "gene_name": "Acetylcholine receptor subunit alpha",
  "term_id": "GO:0043005",
  "gene": "UniProtKB:P02708",
  "gene_symbol": "CHRNA1"
}